{
  "term_label": "serotonin-gated monoatomic cation channel activity",
  "term_id": "GO:0022850",
  "gene": "UniProtKB:Q9UGM1",
  "gene_name": "Neuronal acetylcholine receptor subunit alpha-9",
  "gene_symbol": "CHRNA9"
}